potassium:proton symporter activity [GO:0015387] (molecular function) Definition: Enables the transfer of a solute or solutes from one side of a membrane to the other according to the reaction: K+(out) + H+(out) = K+(in) + H+(in). Sources: TC:2.A.38.-.- Also known as: potassium:hydrogen symporter activity Relationships: is a type of potassium ion transmembrane transporter activity [GO:0015079]; is a type of solute:proton symporter activity [GO:0015295]